{
  "term_id": "GO:0008284",
  "gene": "UniProtKB:P12034",
  "term_label": "positive regulation of cell population proliferation",
  "gene_symbol": "FGF5",
  "gene_name": "Fibroblast growth factor 5"
}